plasminogen activation [GO:0031639] (biological process) References: PMID:9548733 Definition: The process in which inactive plasminogen is processed to active plasmin. This process includes cleavage at an internal Arg-Val site to form an N-terminal A-chain and C-terminal B-chain held together by a disulfide bond, and can include further proteolytic cleavage events to remove the preactivation peptide. Regulation: regulated by regulation of plasminogen activation [GO:0010755]; RO_0002213 by GO:0010756; negatively regulated by negative regulation of plasminogen activation [GO:0010757] Relationships: is a type of zymogen activation [GO:0031638] Also known as: cleavage of plasminogen to plasmin